{
  "term_label": "U2 snRNP",
  "gene": "UniProtKB:Q13435",
  "gene_name": "Splicing factor 3B subunit 2",
  "gene_symbol": "SF3B2",
  "term_id": "GO:0005686"
}